L-tyrosine transmembrane transporter activity [GO:0005302] (MF) Subtypes: GO:0070908 Also known as: L-tyrosine transporter activity, L-tyrosine permease activity, valine/tyrosine/tryptophan permease activity Sources: GOC:ai, GOC:mtg_transport, ISBN:0815340729 Definition: Enables the transfer of L-tyrosine from one side of a membrane to the other. L-tyrosine is 2-amino-3-(4-hydroxyphenyl)propanoic acid. Relationships: is a type of aromatic amino acid transmembrane transporter activity [GO:0015173]; is_a L-amino acid transmembrane transporter activity [GO:0015179]; is part of tyrosine transport [GO:0015828]